{
  "gene_name": "Shugoshin 1",
  "gene": "UniProtKB:Q5FBB7",
  "term_id": "GO:0010457",
  "gene_symbol": "SGO1",
  "term_label": "centriole-centriole cohesion"
}